{
  "term_label": "Unknown cellular component",
  "gene": "UniProtKB:Q9BYS8",
  "term_id": "UNKNOWN:0003",
  "gene_symbol": "LRRC2",
  "gene_name": "Leucine-rich repeat-containing protein 2"
}